{
  "term_id": "GO:0042826",
  "gene_symbol": "BLTP3A",
  "gene": "UniProtKB:Q6BDS2",
  "gene_name": "Bridge-like lipid transfer protein family member 3A",
  "term_label": "histone deacetylase binding"
}